mannosyl-oligosaccharide 1,3-1,6-alpha-mannosidase activity [GO:0004572] (molecular function) Also known as: mannosyl-oligosaccharide (1->3)-(1->6)-alpha-mannosidase activity, mannosyl-oligosaccharide (1->3,6)-alpha-mannosidase activity, mannosyl-oligosaccharide (1->3/6)-alpha-mannosidase activity, ManII activity, mannosidase II activity, 1,3-(1,6-)mannosyl-oligosaccharide alpha-D-mannohydrolase activity, GlcNAc transferase I-dependent alpha1,3[alpha1,6]mannosidase activity, Golgi alpha-mannosidase II, alpha-(1,3/6)-mannosidase activity, alpha-D-mannosidase II, alpha-mannosidase II, exo-1,3-1,6-alpha-mannosidase activity Sources: EC:3.2.1.114 Definition: Catalysis of the hydrolysis of the terminal (1->3)- and (1->6)-linked alpha-D-mannose residues in the mannosyl-oligosaccharide Man(5)(GlcNAc)(3). Relationships: is a type of GO:0015924